{
  "gene_name": "E3 SUMO-protein ligase ZNF451",
  "term_label": "protein sumoylation",
  "gene": "UniProtKB:Q9Y4E5",
  "gene_symbol": "ZNF451",
  "term_id": "GO:0016925"
}